{
  "gene_symbol": "H1-5",
  "gene_name": "Histone H1.5",
  "term_label": "nucleus",
  "gene": "UniProtKB:P16401",
  "term_id": "GO:0005634"
}